type 1A melatonin receptor binding [GO:0031785] (molecular function) Sources: GOC:mah, GOC:nln Relationships: is a type of melatonin receptor binding [GO:0031784] Also known as: type 1A melatonin receptor ligand Definition: Binding to a type 1A melatonin receptor.